{
  "term_id": "UNKNOWN:0003",
  "gene_symbol": "ZNF660",
  "gene": "UniProtKB:Q6AZW8",
  "gene_name": "Zinc finger protein 660",
  "term_label": "Unknown cellular component"
}